{
  "term_label": "intra-Golgi vesicle-mediated transport",
  "term_id": "GO:0006891",
  "gene_name": "Coatomer subunit beta",
  "gene_symbol": "COPB1",
  "gene": "UniProtKB:P53618"
}